{
  "gene_symbol": "VEGFB",
  "gene": "UniProtKB:P49765",
  "term_label": "vascular endothelial growth factor signaling pathway",
  "gene_name": "Vascular endothelial growth factor B",
  "term_id": "GO:0038084"
}